{
  "gene": "UniProtKB:Q9NSU2",
  "term_label": "DNA catabolic process",
  "gene_symbol": "TREX1",
  "term_id": "GO:0006308",
  "gene_name": "Three-prime repair exonuclease 1"
}